{
  "gene": "UniProtKB:Q6UXI7",
  "gene_symbol": "VIT",
  "term_label": "positive regulation of cell-substrate adhesion",
  "gene_name": "Vitrin",
  "term_id": "GO:0010811"
}